{
  "term_label": "protein tyrosine kinase activity",
  "gene": "UniProtKB:P49760",
  "term_id": "GO:0004713",
  "gene_name": "Dual specificity protein kinase CLK2",
  "gene_symbol": "CLK2"
}